{
  "gene": "UniProtKB:Q9H765",
  "term_id": "UNKNOWN:0002",
  "gene_name": "Ankyrin repeat and SOCS box protein 8",
  "gene_symbol": "ASB8",
  "term_label": "Unknown biological process"
}